{
  "term_id": "GO:0000978",
  "gene_name": "Homeobox protein Hox-A6",
  "gene": "UniProtKB:P31267",
  "gene_symbol": "HOXA6",
  "term_label": "RNA polymerase II cis-regulatory region sequence-specific DNA binding"
}